phosphoenolpyruvate carboxykinase (ATP) activity [GO:0004612] (molecular function) Relationships: is a type of phosphoenolpyruvate carboxykinase activity [GO:0004611] Sources: EC:4.1.1.49, RHEA:18617 Also known as: phosphoenolpyruvic carboxykinase, phosphopyruvate carboxykinase, ATP:oxaloacetate carboxy-lyase (transphosphorylating), ATP:oxaloacetate carboxy-lyase (transphosphorylating; phosphoenolpyruvate-forming), PEPCK (ATP), PEPK, phosphoenolpyruvate carboxylase (ATP), phosphopyruvate carboxykinase (adenosine triphosphate), phosphopyruvate carboxylase (ATP) Definition: Catalysis of the reaction: ATP + oxaloacetate = ADP + CO2 + H+ + phosphoenolpyruvate.